penicillin binding [GO:0008658] (molecular function) Definition: Binding to penicillin, an antibiotic that contains the condensed beta-lactamthiazolidine ring system. Relationships: is a type of amide binding [GO:0033218]; is_a GO:0033293; is a type of heterocyclic compound binding [GO:1901363]; is a type of sulfur compound binding [GO:1901681] Sources: GOC:ai